{
  "gene_symbol": "TSNAX",
  "gene_name": "Translin-associated protein X",
  "term_id": "GO:0004521",
  "gene": "UniProtKB:Q99598",
  "term_label": "RNA endonuclease activity"
}